{
  "term_label": "Unknown molecular function",
  "gene": "UniProtKB:P20963",
  "term_id": "UNKNOWN:0001",
  "gene_symbol": "CD247",
  "gene_name": "T-cell surface glycoprotein CD3 zeta chain"
}